negative regulation of antimicrobial peptide production [GO:0002785] (biological process) Definition: Any process that stops, prevents, or reduces the frequency, rate, or extent of antimicrobial peptide production. Relationships: is a type of negative regulation of production of molecular mediator of immune response [GO:0002701]; is a type of regulation of antimicrobial peptide production [GO:0002784]; is a type of GO:0008348; negatively regulates antimicrobial peptide production [GO:0002775] Sources: GOC:add Subtypes: GO:0002787, GO:0002789, negative regulation of antimicrobial peptide secretion [GO:0002795], negative regulation of antimicrobial peptide biosynthetic process [GO:0002806] Also known as: down regulation of antimicrobial peptide production, down-regulation of antimicrobial peptide production, downregulation of antimicrobial peptide production, inhibition of antimicrobial peptide production